{
  "gene_name": "Peroxisomal 2,4-dienoyl-CoA reductase [(3E)-enoyl-CoA-producing]",
  "term_label": "2,4-dienoyl-CoA reductase (NADPH) activity",
  "term_id": "GO:0008670",
  "gene_symbol": "DECR2",
  "gene": "UniProtKB:Q9NUI1"
}